negative regulation of tissue kallikrein-kinin cascade [GO:0002546] (biological process) Relationships: is a type of negative regulation of kinin cascade [GO:0002257]; is a type of GO:0002382; negatively regulates tissue kallikrein-kinin cascade [GO:0002255] Sources: GOC:add Also known as: down regulation of tissue kallikrein-kinin cascade, down-regulation of tissue kallikrein-kinin cascade, downregulation of tissue kallikrein-kinin cascade, negative regulation of glandular kallikrein-kinin cascade, inhibition of tissue kallikrein-kinin cascade Definition: Any process that stops, prevents, or reduces the frequency, rate, or extent of the tissue kallikrein-kinin cascade.